{
  "gene_name": "Serine_threonine-protein kinase 31",
  "gene_symbol": "STK31",
  "term_id": "UNKNOWN:0003",
  "term_label": "Unknown cellular component",
  "gene": "UniProtKB:Q9BXU1"
}